{
  "gene_name": "Coronin-6",
  "gene": "UniProtKB:Q6QEF8",
  "gene_symbol": "CORO6",
  "term_label": "actin filament",
  "term_id": "GO:0005884"
}